{
  "term_id": "GO:0005829",
  "term_label": "cytosol",
  "gene_symbol": "DPYSL4",
  "gene_name": "Dihydropyrimidinase-related protein 4",
  "gene": "UniProtKB:O14531"
}